4-hydroxybenzoate 3-monooxygenase (NADPH) activity [GO:0106356] (molecular function) Definition: Catalysis of the reaction: 4-hydroxybenzoate + H+ + NADPH + O2 = 3,4-dihydroxybenzoate + H2O + NADP+. Sources: RHEA:19477 Relationships: is a type of 4-hydroxybenzoate 3-monooxygenase [NAD(P)H] activity [GO:0018671] Also known as: 4-hydroxybenzoate 3-monooxygenase [NADPH] activity